post-embryonic dorsal fin morphogenesis [GO:0035134] (biological process) Relationships: is a type of post-embryonic medial fin morphogenesis [GO:0035132]; is a type of dorsal fin morphogenesis [GO:0035142] Definition: The process, occurring after embryonic development, by which the anatomical structures of the dorsal fin are generated and organized. A dorsal fin is an unpaired medial fin on the dorsal aspect of a fish that provides lateral stability while swimming. Generally fish have one or two dorsal fins. Sources: GOC:dgh